{
  "gene": "UniProtKB:Q6P988",
  "term_id": "GO:0140776",
  "gene_symbol": "NOTUM",
  "term_label": "protein-containing complex destabilizing activity",
  "gene_name": "Palmitoleoyl-protein carboxylesterase NOTUM"
}